response to antidepressant [GO:0036276] (BP) Subtypes: response to fluoxetine [GO:0014076] Relationships: is a type of response to chemical [GO:0042221] Definition: Any process that results in a change in state or activity of a cell or an organism (in terms of movement, secretion, enzyme production, gene expression, etc.) as a result of an antidepressant stimulus, a mood-stimulating drug. Note: Note that this term is in the subset of terms that should not be used for direct manual annotation of gene products. It was created to be used for cross-referencing by other ontologies. Direct annotations to this term may be amended during annotation QC. Sources: GOC:hp